bicarbonate binding [GO:0071890] (molecular function) Also known as: CHO3- ion binding binding, hydrogencarbonate binding Relationships: is a type of anion binding [GO:0043168] Definition: Binding to bicarbonate ions (CHO3-). Sources: GOC:curators